sialic acid transmembrane transporter activity [GO:0015136] (molecular function) Sources: GOC:jl, GOC:mtg_transport, ISBN:0815340729 Relationships: is a type of carbohydrate derivative transmembrane transporter activity [GO:1901505]; is part of GO:0015739 Definition: Enables the transfer of sialic acid from one side of a membrane to the other. Subtypes: sialate:monoatomic cation symporter activity [GO:0015306], sialic acid:proton symporter activity [GO:0015538]